trabecula morphogenesis [GO:0061383] (biological process) Relationships: is a type of GO:0009653 Subtypes: GO:0061384, bone trabecula morphogenesis [GO:0061430] Definition: The process of shaping a trabecula in an organ. A trabecula is a small, often microscopic, tissue element in the form of a small beam, strut or rod, which generally has a mechanical function. Trabecula are usually but not necessarily, composed of dense collagenous tissue. Sources: GOC:dph